{
  "term_label": "dendritic spine",
  "gene_name": "SLIT-ROBO Rho GTPase-activating protein 2B",
  "gene_symbol": "SRGAP2B",
  "gene": "UniProtKB:P0DMP2",
  "term_id": "GO:0043197"
}